protein-RNA complex remodeling [GO:0110136] (biological process) Definition: The acquisition, loss, or modification of macromolecules within a protein-RNA complex, resulting in the alteration of an existing complex. Also known as: protein-RNA complex remodelling References: PMID:19737519, PMID:20542003, PMID:24240281 Sources: GOC:rn Relationships: is a type of protein-containing complex remodeling [GO:0034367]; is a type of protein-RNA complex organization [GO:0071826]